{
  "term_id": "GO:0099072",
  "term_label": "regulation of postsynaptic membrane neurotransmitter receptor levels",
  "gene_name": "Disks large homolog 4",
  "gene_symbol": "DLG4",
  "gene": "UniProtKB:P78352"
}